{
  "gene_symbol": "TRAPPC2",
  "term_label": "cytoplasm",
  "gene": "UniProtKB:P0DI81",
  "gene_name": "Trafficking protein particle complex subunit 2",
  "term_id": "GO:0005737"
}